{
  "term_id": "GO:0000278",
  "gene_symbol": "PTPN6",
  "gene_name": "Tyrosine-protein phosphatase non-receptor type 6",
  "gene": "UniProtKB:P29350",
  "term_label": "mitotic cell cycle"
}